{
  "gene_symbol": "RPS6KB1",
  "term_id": "GO:0032869",
  "gene_name": "Ribosomal protein S6 kinase beta-1",
  "gene": "UniProtKB:P23443",
  "term_label": "cellular response to insulin stimulus"
}